{
  "term_label": "transcription by RNA polymerase I",
  "gene_symbol": "POLR2L",
  "gene_name": "DNA-directed RNA polymerases I, II, and III subunit RPABC5",
  "gene": "UniProtKB:P62875",
  "term_id": "GO:0006360"
}